{
  "gene": "UniProtKB:P02679",
  "term_id": "GO:0031012",
  "gene_symbol": "FGG",
  "term_label": "extracellular matrix",
  "gene_name": "Fibrinogen gamma chain"
}